{
  "gene_symbol": "RETN",
  "term_id": "UNKNOWN:0001",
  "gene_name": "Resistin",
  "gene": "UniProtKB:Q9HD89",
  "term_label": "Unknown molecular function"
}